{
  "gene_symbol": "A0A1W2PQM1",
  "term_id": "UNKNOWN:0003",
  "gene_name": "Immunoglobulin subtype domain-containing protein",
  "term_label": "Unknown cellular component",
  "gene": "UniProtKB:A0A1W2PQM1"
}